{
  "gene_name": "Serpin B8",
  "term_label": "extracellular space",
  "gene_symbol": "SERPINB8",
  "gene": "UniProtKB:P50452",
  "term_id": "GO:0005615"
}